{
  "gene_symbol": "MMEL1",
  "gene": "UniProtKB:Q495T6",
  "term_id": "GO:0004222",
  "term_label": "metalloendopeptidase activity",
  "gene_name": "Membrane metallo-endopeptidase-like 1"
}